{
  "term_label": "axon",
  "term_id": "GO:0030424",
  "gene_symbol": "NRP2",
  "gene_name": "Neuropilin-2",
  "gene": "UniProtKB:O60462"
}